{
  "gene_symbol": "LY6G6F",
  "term_id": "UNKNOWN:0002",
  "term_label": "Unknown biological process",
  "gene": "UniProtKB:Q5SQ64",
  "gene_name": "Lymphocyte antigen 6 complex locus protein G6f"
}